{
  "gene_name": "Helicase MOV-10",
  "term_id": "GO:0035194",
  "term_label": "regulatory ncRNA-mediated post-transcriptional gene silencing",
  "gene": "UniProtKB:Q9HCE1",
  "gene_symbol": "MOV10"
}